facial nerve morphogenesis [GO:0021610] (biological process) Also known as: CN VII morphogenesis Definition: The process in which the anatomical structure of the facial nerve is generated and organized. This sensory and motor nerve supplies the muscles of facial expression and the expression and taste at the anterior two-thirds of the tongue. The principal branches are the superficial ophthalmic, buccal, palatine and hyomandibular. The main trunk synapses within pterygopalatine ganglion in the parotid gland and this ganglion then gives of nerve branches which supply the lacrimal gland and the mucous secreting glands of the nasal and oral cavities. Relationships: is a type of cranial nerve morphogenesis [GO:0021602]; is part of GO:0021561 Sources: GOC:cls, GOC:dgh, GOC:dph, GOC:jid, GO_REF:0000021